{
  "gene_symbol": "PABPC1L",
  "gene_name": "Polyadenylate-binding protein 1-like",
  "term_id": "GO:0010494",
  "gene": "UniProtKB:Q4VXU2",
  "term_label": "cytoplasmic stress granule"
}